{
  "gene_symbol": "FLRT2",
  "term_id": "UNKNOWN:0001",
  "gene": "UniProtKB:O43155",
  "gene_name": "Leucine-rich repeat transmembrane protein FLRT2",
  "term_label": "Unknown molecular function"
}